hypothalamic tangential migration using cell-axon interactions [GO:0021856] (biological process) Relationships: is a type of hypothalamus cell migration [GO:0021855] Definition: The movement of a hypothalamic neuronal precursor tangentially through the forebrain using an interaction of the migrating cells with axons of other neurons. Sources: GOC:cls, GOC:dgh, GOC:dph, GOC:jid, GO_REF:0000021 Subtypes: gonadotrophin-releasing hormone neuronal migration to the hypothalamus [GO:0021828]